{
  "term_label": "Unknown biological process",
  "gene_symbol": "NIT1",
  "gene": "UniProtKB:Q86X76",
  "gene_name": "Deaminated glutathione amidase",
  "term_id": "UNKNOWN:0002"
}